{
  "gene": "UniProtKB:P61073",
  "term_id": "GO:0007204",
  "gene_name": "C-X-C chemokine receptor type 4",
  "term_label": "positive regulation of cytosolic calcium ion concentration",
  "gene_symbol": "CXCR4"
}